geissoschizine dehydrogenase activity [GO:0047920] (molecular function) Relationships: is a type of oxidoreductase activity, acting on the CH-CH group of donors, NAD or NADP as acceptor [GO:0016628] Sources: EC:1.3.1.36, RHEA:11376 Definition: Catalysis of the reaction: geissoschizine + NADP+ = 4,21-dehydrogeissoschizine + H+ + NADPH. Also known as: geissoschizine:NADP+ 4,21-oxidoreductase activity